catabolic process [GO:0009056] (biological process) Also known as: breakdown of chemical, breakdown of molecule, breakdown of substance, catabolism, cellular breakdown, cellular catabolism, cellular degradation, degradation Definition: A cellular process consisting of the biochemical pathways by which a living organism breaks down substances. This includes the breakdown of carbon compounds with the liberation of energy for use by the cell or organism. Relationships: is a type of metabolic process [GO:0008152] Subtypes: GO:0006581, GO:0006798, autophagy [GO:0006914], GO:0009057, amino acid catabolic process [GO:0009063], amine catabolic process [GO:0009310], toxin catabolic process [GO:0009407], cyanate catabolic process [GO:0009440], alkaloid catabolic process [GO:0009822], ureide catabolic process [GO:0010136], bradykinin catabolic process [GO:0010815], lipid catabolic process [GO:0016042], carbohydrate catabolic process [GO:0016052], GO:0017001, 1,2,4-trichlorobenzene catabolic process [GO:0018911], chlorobenzene catabolic process [GO:0018914], GO:0018968, 1,4-dichlorobenzene catabolic process [GO:0019261], phenol-containing compound catabolic process [GO:0019336], cyanide catabolic process [GO:0019500], nicotine catabolic process [GO:0019608], GO:0019700, collagen catabolic process [GO:0030574], tetrapyrrole catabolic process [GO:0033015], nucleobase-containing compound catabolic process [GO:0034655], xenobiotic catabolic process [GO:0042178], GO:0042193, modified amino acid catabolic process [GO:0042219], GO:0042436, hormone catabolic process [GO:0042447], pteridine-containing compound catabolic process [GO:0042560], flavin-containing compound catabolic process [GO:0042728], GO:0042744, beta-ketoadipate pathway [GO:0042952], peptide catabolic process [GO:0043171], nitrate catabolic process [GO:0043602], GO:0043605, sulfur compound catabolic process [GO:0044273], small molecule catabolic process [GO:0044282], nucleobase catabolic process [GO:0046113], GO:0046153, aldehyde catabolic process [GO:0046185], nitric oxide catabolic process [GO:0046210], phenylpropanoid catabolic process [GO:0046271], GO:0046275, GO:0046302, Z-phenylacetaldoxime catabolic process [GO:0046308], GO:0046434, depsipeptide catabolic process [GO:0050762], GO:0050899, GO:0051190, chitobiose catabolic process [GO:0052781], GO:0052805, lactam catabolic process [GO:0072340], GO:0072491, purine-containing compound catabolic process [GO:0072523], pyridine-containing compound catabolic process [GO:0072526], pyrimidine-containing compound catabolic process [GO:0072529], secondary metabolite catabolic process [GO:0090487], hydrocarbon catabolic process [GO:0120253], olefinic compound catabolic process [GO:0120256], amyloid-beta clearance by cellular catabolic process [GO:0150094], austinol catabolic process [GO:1900559], nitrobenzene catabolic process [GO:1900998], bacitracin A catabolic process [GO:1901123], candicidin catabolic process [GO:1901126], carbohydrate derivative catabolic process [GO:1901136], primary amino compound catabolic process [GO:1901161], GO:1901276, iron-sulfur-molybdenum cofactor catabolic process [GO:1901287], lactone catabolic process [GO:1901335], ether catabolic process [GO:1901502], phosphinothricin catabolic process [GO:1901765], 7,8-didemethyl-8-hydroxy-5-deazariboflavin catabolic process [GO:1901851], GO:1901903, betaine aldehyde catabolic process [GO:1902062] Regulation: regulated by GO:0009894; negatively regulated by negative regulation of catabolic process [GO:0009895]; positively regulated by positive regulation of catabolic process [GO:0009896] Sources: ISBN:0198547684